{
  "term_label": "RNA polymerase II, core complex",
  "gene_symbol": "POLR2J",
  "gene": "UniProtKB:P52435",
  "gene_name": "DNA-directed RNA polymerase II subunit RPB11-a",
  "term_id": "GO:0005665"
}